glucuronate isomerase activity [GO:0008880] (molecular function) Also known as: D-glucuronate aldose-ketose-isomerase activity, D-glucuronate isomerase activity, D-glucuronate ketol-isomerase activity, uronate isomerase activity, uronic acid isomerase activity, uronic isomerase activity Definition: Catalysis of the reaction: D-glucuronate = D-fructuronate. Also converts D-galacturonate to D-tagaturonate. Sources: EC:5.3.1.12 Relationships: is a type of intramolecular oxidoreductase activity, interconverting aldoses and ketoses [GO:0016861]